regulation of thyroid-stimulating hormone secretion [GO:2000612] (biological process) Relationships: is_a regulation of peptide hormone secretion [GO:0090276]; regulates GO:0070460 Sources: GOC:obol Subtypes: GO:2000613, GO:2000614 Definition: Any process that modulates the frequency, rate or extent of thyroid-stimulating hormone secretion. Also known as: regulation of TSH secretion, regulation of thyroid stimulating hormone secretion